{
  "term_label": "regulation of circadian rhythm",
  "gene_name": "Serine_threonine-protein phosphatase PP1-alpha catalytic subunit",
  "gene": "UniProtKB:P62136",
  "term_id": "GO:0042752",
  "gene_symbol": "PPP1CA"
}